{
  "gene": "UniProtKB:Q8IVN3",
  "term_label": "Unknown molecular function",
  "gene_name": "Musculoskeletal embryonic nuclear protein 1",
  "gene_symbol": "MUSTN1",
  "term_id": "UNKNOWN:0001"
}